{
  "gene": "UniProtKB:Q96CM3",
  "term_id": "GO:0009982",
  "gene_symbol": "RPUSD4",
  "gene_name": "Pseudouridylate synthase RPUSD4, mitochondrial",
  "term_label": "pseudouridine synthase activity"
}